MIH complex [GO:0120155] (cellular component) Also known as: Mlc1p-Iqg1p-Hof1p complex Definition: A trimeric complex involved in cytokinesis. Proposed to bridge actomyosin ring contraction and septum synthesis in yeast, resulting in the coordination of these processes, and leading to plasma membrane ingression and fusion. In the yeast Saccharomyces cerevisiae this complex consists of Mlc1p, Iqg1p and Hof1p proteins. Relationships: is a type of protein-containing complex [GO:0032991]; is part of cellular bud neck [GO:0005935] References: PMID:24413167, PMID:24895401 Sources: GOC:rn